{
  "term_label": "Unknown molecular function",
  "term_id": "UNKNOWN:0001",
  "gene_name": "ARL14 effector protein",
  "gene_symbol": "ARL14EP",
  "gene": "UniProtKB:Q8N8R7"
}